{
  "gene_name": "Claudin-6",
  "gene_symbol": "CLDN6",
  "term_label": "virus receptor activity",
  "gene": "UniProtKB:P56747",
  "term_id": "GO:0001618"
}